{
  "gene": "UniProtKB:Q92887",
  "term_id": "GO:0005886",
  "term_label": "plasma membrane",
  "gene_symbol": "ABCC2",
  "gene_name": "ATP-binding cassette sub-family C member 2"
}